{
  "gene": "UniProtKB:O60667",
  "gene_symbol": "FCMR",
  "term_label": "plasma membrane",
  "gene_name": "Fas apoptotic inhibitory molecule 3",
  "term_id": "GO:0005886"
}